{
  "gene_name": "Transmembrane protein 130",
  "term_label": "plasma membrane",
  "gene": "UniProtKB:Q8N3G9",
  "gene_symbol": "TMEM130",
  "term_id": "GO:0005886"
}